{
  "gene_symbol": "NBPF14",
  "term_id": "UNKNOWN:0002",
  "gene": "UniProtKB:Q5TI25",
  "gene_name": "Neuroblastoma breakpoint family member 14",
  "term_label": "Unknown biological process"
}